{
  "gene": "UniProtKB:Q9BYV9",
  "gene_name": "Transcription regulator protein BACH2",
  "term_id": "UNKNOWN:0003",
  "term_label": "Unknown cellular component",
  "gene_symbol": "BACH2"
}